{
  "gene": "UniProtKB:Q9BZP3",
  "term_label": "Unknown cellular component",
  "gene_symbol": "LINC00470",
  "gene_name": "Putative uncharacterized protein encoded by LINC00470",
  "term_id": "UNKNOWN:0003"
}